{
  "term_label": "metalloendopeptidase activity",
  "gene_symbol": "ZMPSTE24",
  "gene_name": "CAAX prenyl protease 1 homolog",
  "term_id": "GO:0004222",
  "gene": "UniProtKB:O75844"
}